{
  "gene_symbol": "MTIF3",
  "gene": "UniProtKB:Q9H2K0",
  "term_label": "mitochondrial translational initiation",
  "gene_name": "Translation initiation factor IF-3, mitochondrial",
  "term_id": "GO:0070124"
}